{
  "gene_symbol": "DCUN1D3",
  "gene": "UniProtKB:Q8IWE4",
  "term_id": "GO:0000151",
  "gene_name": "DCN1-like protein 3",
  "term_label": "ubiquitin ligase complex"
}